complement activation, alternative pathway [GO:0006957] (biological process) Regulation: regulated by regulation of complement activation, alternative pathway [GO:0030451]; negatively regulated by GO:0045957; positively regulated by positive regulation of complement activation, alternative pathway [GO:0045958] Sources: GOC:add, ISBN:0781735149 Relationships: is a type of complement activation [GO:0006956]; is_a innate immune response [GO:0045087] Definition: Any process involved in the activation of any of the steps of the alternative pathway of the complement cascade which allows for the direct killing of microbes and the regulation of other immune processes. Also known as: complement cascade, alternative pathway